{
  "gene_symbol": "PDZRN4",
  "gene_name": "PDZ domain-containing RING finger protein 4",
  "term_id": "UNKNOWN:0001",
  "term_label": "Unknown molecular function",
  "gene": "UniProtKB:Q6ZMN7"
}